{
  "gene_name": "CCR4-NOT transcription complex subunit 10",
  "gene": "UniProtKB:Q9H9A5",
  "gene_symbol": "CNOT10",
  "term_label": "CCR4-NOT complex",
  "term_id": "GO:0030014"
}